{
  "gene": "UniProtKB:Q68DU8",
  "term_id": "GO:0042734",
  "gene_name": "BTB_POZ domain-containing protein KCTD16",
  "term_label": "presynaptic membrane",
  "gene_symbol": "KCTD16"
}